RNA polymerase II, holoenzyme [GO:0016591] (cellular component) Definition: A nuclear DNA-directed RNA polymerase complex containing an RNA polymerase II core enzyme as well as additional proteins and transcription factor complexes, that are capable of promoter recognition and transcription initiation from an RNA polymerase II promoter in vivo. These additional components may include general transcription factor complexes TFIIA, TFIID, TFIIE, TFIIF, or TFIIH, as well as Mediator, SWI/SNF, GCN5, or SRBs and confer the ability to recognize promoters. Also known as: DNA-directed RNA polymerase II, holoenzyme Relationships: is a type of nuclear DNA-directed RNA polymerase complex [GO:0055029] References: PMID:16858867 Sources: GOC:jl, GOC:krc, Wikipedia:Rna_polymerase_ii